apolipoprotein A-I receptor activity [GO:0034188] (molecular function) References: PMID:16443932 Sources: GOC:BHF, GOC:bf, GOC:rl, GOC:signaling Relationships: is a type of GO:0004888; is a type of apolipoprotein receptor activity [GO:0030226]; BFO_0000050 apolipoprotein A-I-mediated signaling pathway [GO:0038027]; has part apolipoprotein A-I binding [GO:0034186] Definition: Combining with an apolipoprotein A-I receptor ligand and transmitting the signal from one side of the membrane to the other to initiate a change in cell activity.